{
  "term_label": "RNA polymerase II cis-regulatory region sequence-specific DNA binding",
  "gene": "UniProtKB:Q8N7M2",
  "term_id": "GO:0000978",
  "gene_name": "Zinc finger protein 283",
  "gene_symbol": "ZNF283"
}